{
  "term_label": "Unknown molecular function",
  "term_id": "UNKNOWN:0001",
  "gene_name": "14-3-3 protein theta",
  "gene_symbol": "YWHAQ",
  "gene": "UniProtKB:P27348"
}